{
  "gene_symbol": "GSK3B",
  "term_id": "GO:0005634",
  "term_label": "nucleus",
  "gene": "UniProtKB:P49841",
  "gene_name": "Glycogen synthase kinase-3 beta"
}